{
  "term_id": "UNKNOWN:0001",
  "term_label": "Unknown molecular function",
  "gene": "UniProtKB:P62910",
  "gene_name": "Large ribosomal subunit protein eL32",
  "gene_symbol": "RPL32"
}